mitotic cell cycle phase transition [GO:0044772] (biological process) Relationships: is a type of GO:0044770; is_a mitotic cell cycle process [GO:1903047] Sources: GOC:mtg_cell_cycle Regulation: RO_0002211 by GO:1901990; negatively regulated by negative regulation of mitotic cell cycle phase transition [GO:1901991]; positively regulated by positive regulation of mitotic cell cycle phase transition [GO:1901992] Subtypes: G1/S transition of mitotic cell cycle [GO:0000082], G2/M transition of mitotic cell cycle [GO:0000086], metaphase/anaphase transition of mitotic cell cycle [GO:0007091], exit from mitosis [GO:0010458] Definition: The cell cycle process by which a cell commits to entering the next mitotic cell cycle phase.